collagen type II trimer [GO:0005585] (cellular component) References: PMID:21421911 Relationships: is a type of fibrillar collagen trimer [GO:0005583] Definition: A collagen homotrimer of alpha1(II) chains; type II collagen triple helices associate to form fibrils.